{
  "gene": "UniProtKB:Q05639",
  "term_label": "GTPase activity",
  "gene_symbol": "EEF1A2",
  "gene_name": "Elongation factor 1-alpha 2",
  "term_id": "GO:0003924"
}